{
  "term_id": "UNKNOWN:0001",
  "term_label": "Unknown molecular function",
  "gene_symbol": "G0S2",
  "gene": "UniProtKB:P27469",
  "gene_name": "G0_G1 switch protein 2"
}